{
  "gene_symbol": "CHRNA5",
  "term_label": "neuron projection",
  "gene_name": "Neuronal acetylcholine receptor subunit alpha-5",
  "term_id": "GO:0043005",
  "gene": "UniProtKB:P30532"
}